{
  "gene_name": "Neural retina-specific leucine zipper protein",
  "term_id": "GO:0006357",
  "term_label": "regulation of transcription by RNA polymerase II",
  "gene": "UniProtKB:P54845",
  "gene_symbol": "NRL"
}